hydroperoxide reductase activity [GO:0032843] (molecular function) Definition: Catalysis of the reaction: 2 RSH + ROOH = RSSR + ROH + H2O. This reaction is the thiol-dependent conversion of an organic hydroperoxide to the corresponding alcohol. References: PMID:12540833 Sources: GOC:mlg Relationships: is a type of oxidoreductase activity, acting on a sulfur group of donors, disulfide as acceptor [GO:0016671]